{
  "gene": "UniProtKB:Q16690",
  "gene_name": "Dual specificity protein phosphatase 5",
  "term_id": "GO:0001706",
  "term_label": "endoderm formation",
  "gene_symbol": "DUSP5"
}